{
  "gene": "UniProtKB:Q8N461",
  "gene_symbol": "FBXL16",
  "term_label": "SCF ubiquitin ligase complex",
  "term_id": "GO:0019005",
  "gene_name": "F-box_LRR-repeat protein 16"
}